glutamin-(asparagin-)ase activity [GO:0050417] (molecular function) Definition: Catalysis of the reaction: H2O + L-glutamine = NH3 + L-glutamate; and H2O + L-asparagine = NH3 + L-aspartate. Sources: EC:3.5.1.38 Also known as: glutaminase-(asparagin-)ase activity, L-ASNase/L-GLNase activity, L-asparagine/L-glutamine amidohydrolase activity, L-glutamine(L-asparagine) amidohydrolase activity, glutaminase-asparaginase activity Relationships: is a type of GO:0016811